{
  "term_label": "regulation of cell shape",
  "gene_symbol": "RAC1",
  "gene": "UniProtKB:P63000",
  "gene_name": "Ras-related C3 botulinum toxin substrate 1",
  "term_id": "GO:0008360"
}